regulation of mast cell differentiation [GO:0060375] (biological process) Definition: Any process that modulates the rate, frequency or extent of mast cell differentiation, the process in which a relatively unspecialized myeloid precursor cell acquires the specialized features of a mast cell. A mast cell is a cell that is found in almost all tissues containing numerous basophilic granules and capable of releasing large amounts of histamine and heparin upon activation. Subtypes: positive regulation of mast cell differentiation [GO:0060376], negative regulation of mast cell differentiation [GO:0060377] Relationships: is a type of GO:0002761; regulates mast cell differentiation [GO:0060374] Sources: GOC:dph, GOC:tb